{
  "gene_symbol": "PODXL",
  "gene_name": "Podocalyxin",
  "term_id": "GO:0033634",
  "gene": "UniProtKB:O00592",
  "term_label": "positive regulation of cell-cell adhesion mediated by integrin"
}